{
  "gene_symbol": "PRAMEF12",
  "term_label": "cytoplasm",
  "term_id": "GO:0005737",
  "gene": "UniProtKB:O95522",
  "gene_name": "PRAME family member 12"
}